{
  "term_id": "GO:0007399",
  "gene": "UniProtKB:Q9UHC6",
  "term_label": "nervous system development",
  "gene_name": "Contactin-associated protein-like 2",
  "gene_symbol": "CNTNAP2"
}